branching involved in ureteric bud morphogenesis [GO:0001658] (biological process) Regulation: regulated by regulation of branching involved in ureteric bud morphogenesis [GO:0090189]; positively regulated by positive regulation of branching involved in ureteric bud morphogenesis [GO:0090190]; negatively regulated by negative regulation of branching involved in ureteric bud morphogenesis [GO:0090191] Also known as: ureteric bud branching Definition: The process in which the branching structure of the ureteric bud is generated and organized. The ureteric bud is an epithelial tube that grows out from the metanephric duct. The bud elongates and branches to give rise to the ureter and kidney collecting tubules. Relationships: is a type of branching morphogenesis of an epithelial tube [GO:0048754]; is part of GO:0060675 References: PMID:16916378 Sources: GOC:dph